{
  "term_label": "gap junction channel activity",
  "gene_name": "Gap junction beta-7 protein",
  "gene": "UniProtKB:Q6PEY0",
  "gene_symbol": "GJB7",
  "term_id": "GO:0005243"
}